evoked excitatory postsynaptic potential [GO:0098817] (biological process) Definition: A process that leads to a temporary increase in postsynaptic potential due to the flow of positively charged ions into the postsynaptic cell induced by the evoked release of many vesicles of excitatory neurotransmitter at the synapse. Relationships: is a type of excitatory postsynaptic potential [GO:0060079] Sources: GOC:dos